{
  "gene_name": "GTPase ERas",
  "term_label": "GTPase activity",
  "gene": "UniProtKB:Q7Z444",
  "gene_symbol": "ERAS",
  "term_id": "GO:0003924"
}